{
  "term_id": "GO:0048471",
  "gene": "UniProtKB:P39687",
  "gene_symbol": "ANP32A",
  "term_label": "perinuclear region of cytoplasm",
  "gene_name": "Acidic leucine-rich nuclear phosphoprotein 32 family member A"
}